{
  "term_id": "GO:0043138",
  "gene": "UniProtKB:P46063",
  "gene_symbol": "RECQL",
  "gene_name": "ATP-dependent DNA helicase Q1",
  "term_label": "3'-5' DNA helicase activity"
}